{
  "gene": "UniProtKB:Q9ULA0",
  "term_label": "Unknown cellular component",
  "gene_symbol": "DNPEP",
  "gene_name": "Aspartyl aminopeptidase",
  "term_id": "UNKNOWN:0003"
}